{
  "gene": "UniProtKB:Q96FT9",
  "term_id": "GO:0030991",
  "gene_name": "Intraflagellar transport protein 43 homolog",
  "term_label": "intraciliary transport particle A",
  "gene_symbol": "IFT43"
}